multicellular organism adhesion [GO:0022608] (biological process) Relationships: is a type of multicellular organismal process [GO:0032501] Definition: The attachment of a multicellular organism to a substrate or other organism. Subtypes: multicellular organism adhesion to substrate [GO:0022609] Sources: GOC:isa_complete